{
  "gene_name": "Slit homolog 3 protein",
  "term_label": "Roundabout binding",
  "gene": "UniProtKB:O75094",
  "term_id": "GO:0048495",
  "gene_symbol": "SLIT3"
}